{
  "term_label": "Unknown biological process",
  "gene": "UniProtKB:A6NM11",
  "gene_name": "Leucine-rich repeat-containing protein 37A2",
  "gene_symbol": "LRRC37A2",
  "term_id": "UNKNOWN:0002"
}